{
  "term_label": "protein phosphatase regulator activity",
  "gene": "UniProtKB:Q9Y5P8",
  "term_id": "GO:0019888",
  "gene_symbol": "PPP2R3B",
  "gene_name": "Serine_threonine-protein phosphatase 2A regulatory subunit B'' subunit beta"
}